acireductone dioxygenase (Ni2+-requiring) activity [GO:0010308] (molecular function) Relationships: is a type of oxidoreductase activity, acting on single donors with incorporation of molecular oxygen, incorporation of two atoms of oxygen [GO:0016702] Sources: EC:1.13.11.53, RHEA:14161 Also known as: 2-hydroxy-3-keto-5-thiomethylpent-1-ene dioxygenase activity, acireductone dioxygenase activity, 1,2-dihydroxy-5-(methylthio)pent-1-en-3-one:oxygen oxidoreductase (formate- and CO-forming), ARD activity, E-2 activity Definition: Catalysis of the reaction: 1,2-dihydroxy-5-(methylthio)pent-1-en-3-one + O2 = 3-(methylthio)propanoate + CO + formate.